{
  "gene_symbol": "RPL17",
  "gene": "UniProtKB:P18621",
  "term_label": "cytoplasmic translation",
  "term_id": "GO:0002181",
  "gene_name": "Large ribosomal subunit protein uL22"
}